{
  "gene": "UniProtKB:Q8WVR3",
  "term_label": "cilium assembly",
  "gene_symbol": "TRAPPC14",
  "term_id": "GO:0060271",
  "gene_name": "Trafficking protein particle complex subunit 14"
}